{
  "term_id": "GO:0098609",
  "term_label": "cell-cell adhesion",
  "gene_symbol": "CD2",
  "gene_name": "T-cell surface antigen CD2",
  "gene": "UniProtKB:P06729"
}